{
  "gene_symbol": "TEX13D",
  "term_label": "Unknown cellular component",
  "gene": "UniProtKB:A0A0J9YY54",
  "term_id": "UNKNOWN:0003",
  "gene_name": "Testis-expressed protein 13D"
}